{
  "term_id": "GO:0009897",
  "gene": "UniProtKB:O00421",
  "term_label": "external side of plasma membrane",
  "gene_name": "C-C chemokine receptor-like 2",
  "gene_symbol": "CCRL2"
}